{
  "gene": "UniProtKB:O60506",
  "gene_name": "Heterogeneous nuclear ribonucleoprotein Q",
  "term_id": "GO:1990904",
  "gene_symbol": "SYNCRIP",
  "term_label": "ribonucleoprotein complex"
}